regulation of exosomal secretion [GO:1903541] (biological process) Subtypes: negative regulation of exosomal secretion [GO:1903542], positive regulation of exosomal secretion [GO:1903543] Relationships: is a type of regulation of exocytosis [GO:0017157]; regulates exosomal secretion [GO:1990182] References: PMID:24105262 Sources: GOC:TermGenie, GO_REF:0000058 Also known as: regulation of exosomal secretory pathway, regulation of extracellular vesicular exosome secretion, regulation of secretion of exosome, regulation of exosomal protein secretion Definition: Any process that modulates the frequency, rate or extent of exosomal secretion.